{
  "term_label": "RNA polymerase II cis-regulatory region sequence-specific DNA binding",
  "gene_name": "Forkhead box protein B1",
  "gene_symbol": "FOXB1",
  "gene": "UniProtKB:Q99853",
  "term_id": "GO:0000978"
}